{
  "term_id": "GO:0006959",
  "gene_name": "Immunoglobulin J chain",
  "term_label": "humoral immune response",
  "gene": "UniProtKB:P01591",
  "gene_symbol": "JCHAIN"
}